{
  "gene_name": "Tenomodulin",
  "gene_symbol": "TNMD",
  "term_id": "UNKNOWN:0003",
  "gene": "UniProtKB:Q9H2S6",
  "term_label": "Unknown cellular component"
}